{
  "gene_name": "Stanniocalcin-2",
  "gene_symbol": "STC2",
  "term_id": "UNKNOWN:0001",
  "term_label": "Unknown molecular function",
  "gene": "UniProtKB:O76061"
}